geranial dehydrogenase activity [GO:0034832] (molecular function) Relationships: is a type of oxidoreductase activity, acting on the aldehyde or oxo group of donors, NAD or NADP as acceptor [GO:0016620] Sources: RHEA:34351 Definition: Catalysis of the reaction: (2E)-geranial + H2O + NAD+ = geranate + 2 H+ + NADH.